juvenile hormone biosynthetic process [GO:0006718] (biological process) Sources: GOC:go_curators, ISBN:0198547684 Relationships: is a type of GO:0006716; is a type of sesquiterpenoid biosynthetic process [GO:0016106]; is a type of hormone biosynthetic process [GO:0042446] Also known as: juvenile hormone anabolism, juvenile hormone biosynthesis, juvenile hormone formation, juvenile hormone synthesis Regulation: regulated by regulation of juvenile hormone biosynthetic process [GO:0007557]; negatively regulated by negative regulation of juvenile hormone biosynthetic process [GO:0045968]; positively regulated by GO:0045969 Definition: The chemical reactions and pathways resulting in the formation of juvenile hormones, the three sesquiterpenoid derivatives that function to maintain the larval state of insects at molting and that may be required for other processes, e.g. oogenesis.